{
  "gene_symbol": "OR2W3",
  "gene_name": "Olfactory receptor 2W3",
  "gene": "UniProtKB:Q7Z3T1",
  "term_label": "plasma membrane",
  "term_id": "GO:0005886"
}